{
  "gene_symbol": "CD55",
  "gene": "UniProtKB:P08174",
  "term_label": "Unknown biological process",
  "term_id": "UNKNOWN:0002",
  "gene_name": "Complement decay-accelerating factor"
}